regulation of single-species biofilm formation in or on host organism [GO:1900228] (biological process) Subtypes: negative regulation of single-species biofilm formation in or on host organism [GO:1900229], positive regulation of single-species biofilm formation in or on host organism [GO:1900230] Relationships: is a type of regulation of biological process involved in symbiotic interaction [GO:0043903]; is a type of regulation of single-species biofilm formation [GO:1900190]; regulates single-species biofilm formation in or on host organism [GO:0044407] Sources: GOC:TermGenie, GOC:di Definition: Any process that modulates the frequency, rate or extent of single-species biofilm formation in or on host organism.